{
  "gene": "UniProtKB:P33176",
  "term_id": "GO:0098971",
  "gene_symbol": "KIF5B",
  "gene_name": "Kinesin-1 heavy chain",
  "term_label": "anterograde dendritic transport of neurotransmitter receptor complex"
}